{
  "term_label": "exocytosis",
  "gene_name": "Exocyst complex component 3-like protein",
  "term_id": "GO:0006887",
  "gene": "UniProtKB:Q86VI1",
  "gene_symbol": "EXOC3L1"
}